regulation of cysteine metabolic process [GO:1901494] (BP) Relationships: is a type of regulation of amino acid metabolic process [GO:0006521]; is a type of regulation of sulfur metabolic process [GO:0042762]; is a type of regulation of small molecule metabolic process [GO:0062012]; regulates cysteine metabolic process [GO:0006534] Sources: GOC:TermGenie Definition: Any process that modulates the frequency, rate or extent of cysteine metabolic process. Also known as: regulation of cysteine metabolism